{
  "gene": "UniProtKB:P09497",
  "gene_name": "Clathrin light chain B",
  "term_id": "GO:0072583",
  "gene_symbol": "CLTB",
  "term_label": "clathrin-dependent endocytosis"
}